{
  "gene_name": "Cell surface glycoprotein CD200 receptor 2",
  "term_id": "GO:0038023",
  "gene": "UniProtKB:Q6Q8B3",
  "gene_symbol": "CD200R1L",
  "term_label": "signaling receptor activity"
}